{
  "gene_symbol": "XBP1",
  "gene_name": "X-box-binding protein 1",
  "gene": "UniProtKB:P17861",
  "term_label": "RNA polymerase II transcription regulatory region sequence-specific DNA binding",
  "term_id": "GO:0000977"
}